{
  "gene_name": "Methionine-R-sulfoxide reductase B2, mitochondrial",
  "gene_symbol": "MSRB2",
  "term_label": "peptide-methionine (R)-S-oxide reductase activity",
  "gene": "UniProtKB:Q9Y3D2",
  "term_id": "GO:0033743"
}